FMN reductase (NADH) activity [GO:0052874] (MF) Sources: RHEA:21620 Relationships: is a type of FMN reductase [NAD(P)H] activity [GO:0008752] Also known as: NADH dehydrogenase (FMN) activity, NADH-FMN reductase activity, NADH-dependent FMN reductase activity Definition: Catalysis of the reaction: FMNH2 + NAD+ = FMN + NADH + 2 H+.